{
  "gene_name": "Zinc finger protein with KRAB and SCAN domains 2",
  "gene": "UniProtKB:Q63HK3",
  "term_label": "DNA-binding transcription factor activity, RNA polymerase II-specific",
  "term_id": "GO:0000981",
  "gene_symbol": "ZKSCAN2"
}